{
  "gene": "UniProtKB:P60201",
  "term_label": "myelin sheath",
  "gene_symbol": "PLP1",
  "term_id": "GO:0043209",
  "gene_name": "Myelin proteolipid protein"
}